{
  "gene_name": "Solute carrier family 22 member 12",
  "term_label": "organic anion transport",
  "term_id": "GO:0015711",
  "gene": "UniProtKB:Q96S37",
  "gene_symbol": "SLC22A12"
}